integrin alphaE-beta7 complex [GO:0034691] (cellular component) Also known as: Itgae-Itgb7 complex Relationships: is a type of integrin complex [GO:0008305] Definition: An integrin complex that comprises one alphaE subunit and one beta7 subunit. References: PMID:12297042